{
  "gene": "UniProtKB:P11169",
  "term_id": "GO:0005886",
  "gene_name": "Solute carrier family 2, facilitated glucose transporter member 3",
  "term_label": "plasma membrane",
  "gene_symbol": "SLC2A3"
}